{
  "term_label": "negative regulation of actin filament depolymerization",
  "gene_symbol": "PLEKHH2",
  "gene_name": "Pleckstrin homology domain-containing family H member 2",
  "term_id": "GO:0030835",
  "gene": "UniProtKB:Q8IVE3"
}